beta-alanine biosynthetic process via 1,3 diaminopropane [GO:0033394] (biological process) Definition: The chemical reactions and pathways resulting in the formation of beta-alanine via the intermediate 1,3 diaminopropane. Also known as: beta-alanine anabolism via 1,3 diaminopropane, beta-alanine biosynthesis via 1,3 diaminopropane, beta-alanine formation via 1,3 diaminopropane, beta-alanine synthesis via 1,3 diaminopropane Relationships: is a type of beta-alanine biosynthetic process [GO:0019483] Sources: GOC:mah, MetaCyc:PWY-3981